{
  "term_label": "Unknown molecular function",
  "gene": "UniProtKB:P57105",
  "gene_name": "Synaptojanin-2-binding protein",
  "gene_symbol": "SYNJ2BP",
  "term_id": "UNKNOWN:0001"
}